magnesium ion export from mitochondrion [GO:1990616] (biological process) Also known as: magnesium ion efflux from mitochondrion Definition: The directed movement of magnesium ions out of mitochondrial matrix into the cytosol by means of some agent such as a transporter or pore. References: PMID:25585246 Relationships: is a type of mitochondrial magnesium ion transmembrane transport [GO:0045016]